{
  "term_id": "GO:0035243",
  "gene_name": "Protein arginine methyltransferase NDUFAF7, mitochondrial",
  "gene": "UniProtKB:Q7L592",
  "term_label": "protein-arginine omega-N symmetric methyltransferase activity",
  "gene_symbol": "NDUFAF7"
}